{
  "gene": "UniProtKB:Q9UJA3",
  "term_id": "GO:0042555",
  "term_label": "MCM complex",
  "gene_name": "DNA helicase MCM8",
  "gene_symbol": "MCM8"
}